G protein-coupled chemorepellent receptor signaling pathway [GO:0140986] (biological process) Definition: A G protein-coupled receptor signaling pathway initiated by a chemorepellent binding to its receptor on the surface of a target cell, and ending with the regulation of a downstream cellular process, e.g. cytoskeleton reorganization. References: PMID:30462573 Relationships: is a type of G protein-coupled receptor signaling pathway [GO:0007186]